{
  "gene_symbol": "MCC",
  "gene_name": "Colorectal mutant cancer protein",
  "term_id": "GO:0090090",
  "gene": "UniProtKB:P23508",
  "term_label": "negative regulation of canonical Wnt signaling pathway"
}